{
  "gene": "UniProtKB:Q8TE99",
  "gene_name": "2-phosphoxylose phosphatase 1",
  "term_label": "phosphatase activity",
  "gene_symbol": "PXYLP1",
  "term_id": "GO:0016791"
}